{
  "gene": "UniProtKB:Q32MZ4",
  "term_label": "DNA-binding transcription factor activity, RNA polymerase II-specific",
  "gene_name": "Leucine-rich repeat flightless-interacting protein 1",
  "gene_symbol": "LRRFIP1",
  "term_id": "GO:0000981"
}